{
  "gene_symbol": "CORO1B",
  "term_label": "cell migration",
  "term_id": "GO:0016477",
  "gene_name": "Coronin-1B",
  "gene": "UniProtKB:Q9BR76"
}